{
  "term_label": "lipopolysaccharide binding",
  "gene_symbol": "DEFB114",
  "term_id": "GO:0001530",
  "gene_name": "Beta-defensin 114",
  "gene": "UniProtKB:Q30KQ6"
}